{
  "term_label": "Unknown biological process",
  "gene": "UniProtKB:Q96B77",
  "gene_symbol": "TMEM186",
  "gene_name": "Transmembrane protein 186",
  "term_id": "UNKNOWN:0002"
}